{
  "gene": "UniProtKB:Q96GA7",
  "gene_name": "Serine dehydratase-like",
  "term_id": "GO:0006567",
  "gene_symbol": "SDSL",
  "term_label": "L-threonine catabolic process"
}